{
  "gene_symbol": "OR9K2",
  "gene": "UniProtKB:Q8NGE7",
  "term_label": "Unknown biological process",
  "term_id": "UNKNOWN:0002",
  "gene_name": "Olfactory receptor 9K2"
}